{
  "gene": "UniProtKB:P01568",
  "term_label": "natural killer cell activation involved in immune response",
  "gene_symbol": "IFNA21",
  "term_id": "GO:0002323",
  "gene_name": "Interferon alpha-21"
}